{
  "gene_symbol": "TAGLN3",
  "gene_name": "Transgelin-3",
  "gene": "UniProtKB:Q9UI15",
  "term_id": "GO:0051015",
  "term_label": "actin filament binding"
}